labrum morphogenesis [GO:0048716] (biological process) Definition: The process in which the anatomical structures of labrum are generated and organized. Sources: GOC:rc Relationships: is a type of post-embryonic animal morphogenesis [GO:0009886]; BFO_0000050 clypeo-labral disc morphogenesis [GO:0007453]; BFO_0000050 labrum development [GO:0048726]